{
  "gene": "UniProtKB:P51648",
  "term_id": "GO:0005737",
  "term_label": "cytoplasm",
  "gene_symbol": "ALDH3A2",
  "gene_name": "Aldehyde dehydrogenase family 3 member A2"
}